{
  "term_label": "regulation of DNA-templated transcription",
  "gene_symbol": "LIMD1",
  "gene_name": "LIM domain-containing protein 1",
  "term_id": "GO:0006355",
  "gene": "UniProtKB:Q9UGP4"
}